adhesion of symbiont to host [GO:0044406] (biological process) Definition: The attachment of a symbiont to its host via either adhesion molecules, general stickiness, or other mechanisms. The host is defined as the larger of the organisms involved in a symbiotic interaction. Sources: GOC:bf, GOC:cc, GOC:dos, GOC:jl Also known as: adhesion to other organism involved in symbiotic interaction, host adhesion, adhesion to host, adhesion to other organism during symbiotic interaction Relationships: is a type of biological process involved in interaction with host [GO:0051701] Subtypes: single-species biofilm formation in or on host organism [GO:0044407], adhesion of symbiont to host cell [GO:0044650], GO:0075001, adhesion of symbiont to host via host extracellular matrix [GO:0141018]